{
  "gene": "UniProtKB:P68402",
  "gene_symbol": "PAFAH1B2",
  "term_label": "1-alkyl-2-acetylglycerophosphocholine esterase complex",
  "term_id": "GO:0008247",
  "gene_name": "Platelet-activating factor acetylhydrolase IB subunit alpha2"
}